{
  "term_id": "GO:0005789",
  "gene_symbol": "MIA2",
  "gene": "UniProtKB:Q96PC5",
  "gene_name": "Melanoma inhibitory activity protein 2",
  "term_label": "endoplasmic reticulum membrane"
}